{
  "gene_name": "Rhophilin-1",
  "gene_symbol": "RHPN1",
  "term_id": "UNKNOWN:0003",
  "gene": "UniProtKB:Q8TCX5",
  "term_label": "Unknown cellular component"
}